aminodeoxyfutalosine synthase activity [GO:0102573] (molecular function) Relationships: is a type of GO:0016765 Definition: Catalysis of the reaction: 3-[(1-carboxylatovinyl)oxy]benzoate(2-) + S-adenosyl-L-methionine + H2O = aminodeoxyfutalosinate + L-methionine + hydrogencarbonate + H+. Sources: EC:2.5.1.120, GOC:pz